{
  "gene": "UniProtKB:Q0VDE8",
  "gene_symbol": "ADIG",
  "gene_name": "Adipogenin",
  "term_label": "nucleus",
  "term_id": "GO:0005634"
}